{
  "term_label": "cytoplasm",
  "gene_symbol": "PACSIN2",
  "gene": "UniProtKB:Q9UNF0",
  "term_id": "GO:0005737",
  "gene_name": "Protein kinase C and casein kinase substrate in neurons protein 2"
}